11-cis-retinol dehydrogenase (NAD+) activity [GO:0106429] (molecular function) Sources: RHEA:55668 Relationships: is a type of alcohol dehydrogenase (NAD+) activity [GO:0004022] Definition: Catalysis of the reaction: 11-cis-retinol--[retinol-binding protein] + NAD+ = 11-cis-retinal--[retinol-binding protein] + NADH + H+. Also known as: 11-cis-retinol dehydrogenase activity